{
  "gene": "UniProtKB:Q8IV48",
  "term_label": "exonucleolytic trimming to generate mature 3'-end of 5.8S rRNA from tricistronic rRNA transcript (SSU-rRNA, 5.8S rRNA, LSU-rRNA)",
  "gene_name": "3'-5' exoribonuclease 1",
  "term_id": "GO:0000467",
  "gene_symbol": "ERI1"
}